{
  "term_id": "GO:0007166",
  "term_label": "cell surface receptor signaling pathway",
  "gene_name": "Probable non-functional T cell receptor beta variable 7-1",
  "gene": "UniProtKB:A0A0A6YYK4",
  "gene_symbol": "TRBV7-1"
}